{
  "gene_symbol": "CTSL3P",
  "gene_name": "Putative inactive cathepsin L-like protein CTSL3P",
  "term_label": "Unknown biological process",
  "gene": "UniProtKB:Q5NE16",
  "term_id": "UNKNOWN:0002"
}